synapse-associated extracellular matrix [GO:0099535] (cellular component) Definition: The extracellular matrix of the perisynaptic space (the extracellular space adjacent to the synapse) and the synaptic cleft. Sources: GOC:dos Relationships: is a type of GO:0140047 Subtypes: GO:0098966 Also known as: extra-synaptic extracellular matrix, synapse-associated ECM